{
  "gene": "UniProtKB:Q69YG0",
  "gene_symbol": "TMEM42",
  "term_id": "UNKNOWN:0002",
  "gene_name": "Transmembrane protein 42",
  "term_label": "Unknown biological process"
}